{
  "gene": "UniProtKB:Q96NR3",
  "gene_name": "Patched domain-containing protein 1",
  "gene_symbol": "PTCHD1",
  "term_label": "Unknown molecular function",
  "term_id": "UNKNOWN:0001"
}